positive regulation of endothelial cell differentiation [GO:0045603] (biological process) Sources: GOC:go_curators Relationships: is_a positive regulation of epithelial cell differentiation [GO:0030858]; is a type of regulation of endothelial cell differentiation [GO:0045601]; RO_0002213 endothelial cell differentiation [GO:0045446] Definition: Any process that activates or increases the frequency, rate or extent of endothelial cell differentiation. Also known as: up regulation of endothelial cell differentiation, up-regulation of endothelial cell differentiation, upregulation of endothelial cell differentiation, activation of endothelial cell differentiation, stimulation of endothelial cell differentiation Subtypes: positive regulation of blood vessel endothelial cell differentiation [GO:0110058]